purine nucleotide binding [GO:0017076] (molecular function) Subtypes: guanyl nucleotide binding [GO:0019001], GO:0030554, purine deoxyribonucleotide binding [GO:0032554], purine ribonucleotide binding [GO:0032555] Sources: GOC:ai Definition: Binding to a purine nucleotide, a compound consisting of a purine nucleoside esterified with (ortho)phosphate. Relationships: is a type of nucleotide binding [GO:0000166]